{
  "gene_symbol": "AGMO",
  "gene_name": "Alkylglycerol monooxygenase",
  "term_id": "GO:0005783",
  "term_label": "endoplasmic reticulum",
  "gene": "UniProtKB:Q6ZNB7"
}